{
  "term_id": "GO:0005930",
  "term_label": "axoneme",
  "gene_symbol": "TTLL3",
  "gene_name": "Tubulin monoglycylase TTLL3",
  "gene": "UniProtKB:Q9Y4R7"
}